taxoid 7beta-hydroxylase activity [GO:0036239] (molecular function) References: PMID:15157877, PMID:15178487 Sources: EC:1.14.14.182 Definition: Catalysis of the reaction: taxusin + [reduced NADPH-hemoprotein reductase] + O2 = 7beta-hydroxytaxusin + [oxidized NADPH-hemoprotein reductase] + H2O. Also converts 2alpha-hydroxytaxusin to 2alpha,7beta-dihydroxytaxusin. Relationships: is a type of oxidoreductase activity, acting on paired donors, with incorporation or reduction of molecular oxygen, reduced flavin or flavoprotein as one donor, and incorporation of one atom of oxygen [GO:0016712]